{
  "gene_name": "Prostatic acid phosphatase",
  "gene_symbol": "ACP3",
  "term_label": "positive regulation of adenosine receptor signaling pathway",
  "gene": "UniProtKB:P15309",
  "term_id": "GO:0060168"
}